{
  "term_id": "UNKNOWN:0001",
  "term_label": "Unknown molecular function",
  "gene_name": "Distal membrane-arm assembly complex protein 2",
  "gene_symbol": "DMAC2",
  "gene": "UniProtKB:Q9NW81"
}